guanosine-containing compound catabolic process [GO:1901069] (biological process) Definition: The chemical reactions and pathways resulting in the breakdown of guanosine-containing compounds (guanosines). Sources: GOC:TermGenie Relationships: is a type of purine ribonucleoside catabolic process [GO:0046130] Also known as: guanosine-containing compound breakdown, guanosine-containing compound catabolism, guanosine-containing compound degradation, guanosines breakdown, guanosines catabolic process, guanosines catabolism, guanosines degradation Subtypes: guanosine catabolic process [GO:0046115], 7-methylguanosine catabolic process [GO:0046119]